regulation of monodictyphenone biosynthetic process [GO:1900843] (biological process) Definition: Any process that modulates the frequency, rate or extent of monodictyphenone biosynthetic process. Relationships: is a type of regulation of ketone biosynthetic process [GO:0010566]; is a type of regulation of secondary metabolite biosynthetic process [GO:1900376]; regulates monodictyphenone biosynthetic process [GO:1900815] Also known as: regulation of monodictyphenone anabolism, regulation of monodictyphenone biosynthesis, regulation of monodictyphenone formation, regulation of monodictyphenone synthesis Subtypes: negative regulation of monodictyphenone biosynthetic process [GO:1900844], positive regulation of monodictyphenone biosynthetic process [GO:1900845] Sources: GOC:TermGenie, GOC:di